{
  "gene_name": "Ataxin-7",
  "term_label": "Unknown molecular function",
  "gene": "UniProtKB:O15265",
  "gene_symbol": "ATXN7",
  "term_id": "UNKNOWN:0001"
}